anaerobic phenol-containing compound biosynthetic process [GO:0046192] (biological process) Sources: GOC:ai Relationships: is_a anaerobic phenol-containing compound metabolic process [GO:0042215]; is a type of phenol-containing compound biosynthetic process [GO:0046189] Also known as: anaerobic phenol-containing compound anabolism, anaerobic phenol-containing compound biosynthesis, anaerobic phenol-containing compound formation, anaerobic phenol-containing compound synthesis Definition: The chemical reactions and pathways resulting in the formation of a phenol, any compound containing one or more hydroxyl groups directly attached to an aromatic carbon ring, in the absence of oxygen.